kidney epithelium development [GO:0072073] (biological process) Definition: The process whose specific outcome is the progression of an epithelium in the kidney over time, from its formation to the mature structure. An epithelium is a tissue that covers the internal or external surfaces of an anatomical structure. Sources: GOC:mtg_kidney_jan10 Relationships: is a type of epithelium development [GO:0060429]; is part of kidney development [GO:0001822] Subtypes: GO:0072009, renal vesicle development [GO:0072087], mesonephric epithelium development [GO:0072163], nephric duct development [GO:0072176], metanephric epithelium development [GO:0072207]